{
  "gene": "UniProtKB:P62263",
  "gene_name": "Small ribosomal subunit protein uS11",
  "term_id": "GO:0000028",
  "term_label": "ribosomal small subunit assembly",
  "gene_symbol": "RPS14"
}